{
  "gene": "UniProtKB:Q8TCY5",
  "term_id": "GO:0106070",
  "gene_name": "Melanocortin-2 receptor accessory protein",
  "term_label": "regulation of adenylate cyclase-activating G protein-coupled receptor signaling pathway",
  "gene_symbol": "MRAP"
}